{
  "term_id": "GO:0030424",
  "gene_name": "BDNF_NT-3 growth factors receptor",
  "term_label": "axon",
  "gene": "UniProtKB:Q16620",
  "gene_symbol": "NTRK2"
}